{
  "term_label": "cell differentiation",
  "gene_symbol": "EHF",
  "gene": "UniProtKB:Q9NZC4",
  "gene_name": "ETS homologous factor",
  "term_id": "GO:0030154"
}